GINS complex assembly [GO:0071165] (biological process) References: PMID:16990792 Sources: GOC:mah Definition: The aggregation, arrangement and bonding together of a set of components to form a GINS complex, a heterotetrameric protein complex that associates with DNA replication origins and replication forks. Relationships: is a type of DNA replication preinitiation complex assembly [GO:0071163]